{
  "gene_name": "Keratin-associated protein 4-11",
  "term_id": "UNKNOWN:0003",
  "gene_symbol": "KRTAP4-11",
  "term_label": "Unknown cellular component",
  "gene": "UniProtKB:Q9BYQ6"
}